{
  "term_id": "GO:0008076",
  "gene": "UniProtKB:Q8WWG9",
  "gene_symbol": "KCNE4",
  "term_label": "voltage-gated potassium channel complex",
  "gene_name": "Potassium voltage-gated channel subfamily E member 4"
}